{
  "term_id": "GO:0005634",
  "gene": "UniProtKB:P23497",
  "term_label": "nucleus",
  "gene_name": "Nuclear autoantigen Sp-100",
  "gene_symbol": "SP100"
}